negative regulation of endoplasmic reticulum stress-induced neuron intrinsic apoptotic signaling pathway [GO:1903382] (biological process) Definition: Any process that stops, prevents or reduces the frequency, rate or extent of an endoplasmic reticulum stress-induced neuron intrinsic apoptotic signaling pathway. References: PMID:23453807 Sources: GOC:PARL, GOC:TermGenie, GOC:bf, GO_REF:0000058 Relationships: is a type of negative regulation of neuron apoptotic process [GO:0043524]; is a type of negative regulation of endoplasmic reticulum stress-induced intrinsic apoptotic signaling pathway [GO:1902236]; is a type of regulation of endoplasmic reticulum stress-induced neuron intrinsic apoptotic signaling pathway [GO:1903381]; negatively regulates neuron intrinsic apoptotic signaling pathway in response to endoplasmic reticulum stress [GO:0036483] Also known as: down regulation of ER stress-induced neuron intrinsic apoptotic signaling pathway, down regulation of endoplasmic reticulum stress-induced neuron intrinsic apoptotic signaling pathway, down regulation of neuron intrinsic apoptotic signaling pathway in response to endoplasmic reticulum stress, down-regulation of ER stress-induced neuron intrinsic apoptotic signaling pathway, down-regulation of endoplasmic reticulum stress-induced neuron intrinsic apoptotic signaling pathway, down-regulation of neuron intrinsic apoptotic signaling pathway in response to endoplasmic reticulum stress, downregulation of ER stress-induced neuron intrinsic apoptotic signaling pathway, downregulation of endoplasmic reticulum stress-induced neuron intrinsic apoptotic signaling pathway, downregulation of neuron intrinsic apoptotic signaling pathway in response to endoplasmic reticulum stress, negative regulation of ER stress-induced neuron intrinsic apoptotic signaling pathway, negative regulation of neuron intrinsic apoptotic signaling pathway in response to endoplasmic reticulum stress, inhibition of ER stress-induced neuron intrinsic apoptotic signaling pathway, inhibition of endoplasmic reticulum stress-induced neuron intrinsic apoptotic signaling pathway, inhibition of neuron intrinsic apoptotic signaling pathway in response to endoplasmic reticulum stress